tripartite regional subdivision [GO:0007351] (biological process) Sources: GOC:dph, GOC:isa_complete, ISBN:0879694238, http://fly.ebi.ac.uk/allied-data/lk/interactive-fly/aimain/1aahome.htm Definition: Subdivision of the embryo along the anterior/posterior axis into anterior, posterior and terminal regions. Relationships: is a type of regionalization [GO:0003002]; is part of blastoderm segmentation [GO:0007350]